{
  "gene": "UniProtKB:Q9UKG4",
  "term_id": "GO:0055085",
  "gene_symbol": "SLC13A4",
  "term_label": "transmembrane transport",
  "gene_name": "Solute carrier family 13 member 4"
}